{
  "term_id": "GO:0005737",
  "gene": "UniProtKB:P14373",
  "gene_symbol": "TRIM27",
  "term_label": "cytoplasm",
  "gene_name": "Zinc finger protein RFP"
}